{
  "term_id": "GO:0000981",
  "gene_symbol": "KLF10",
  "gene_name": "Krueppel-like factor 10",
  "gene": "UniProtKB:Q13118",
  "term_label": "DNA-binding transcription factor activity, RNA polymerase II-specific"
}